{
  "term_id": "GO:0000307",
  "gene": "UniProtKB:P61024",
  "term_label": "cyclin-dependent protein kinase holoenzyme complex",
  "gene_symbol": "CKS1B",
  "gene_name": "Cyclin-dependent kinases regulatory subunit 1"
}